{
  "gene_name": "G1_S-specific cyclin-E1",
  "term_id": "GO:0005737",
  "term_label": "cytoplasm",
  "gene_symbol": "CCNE1",
  "gene": "UniProtKB:P24864"
}